pronephric distal tubule morphogenesis [GO:0039013] (biological process) Definition: The process in which the anatomical structures of a pronephric nephron distal tubule are generated and organized. A pronephric nephron tubule is an epithelial tube that is part of the pronephros. Relationships: is a type of pronephric nephron tubule morphogenesis [GO:0039008]; is a type of distal tubule morphogenesis [GO:0072156]; is part of pronephric distal tubule development [GO:0035777] Sources: GOC:mtg_kidney_jan10